{
  "term_id": "GO:0006508",
  "gene_symbol": "ADAM11",
  "term_label": "proteolysis",
  "gene": "UniProtKB:O75078",
  "gene_name": "Disintegrin and metalloproteinase domain-containing protein 11"
}